{
  "term_label": "Unknown molecular function",
  "term_id": "UNKNOWN:0001",
  "gene_symbol": "EXOC6B",
  "gene_name": "Exocyst complex component 6B",
  "gene": "UniProtKB:Q9Y2D4"
}